{
  "gene_symbol": "CHRNA3",
  "term_label": "acetylcholine-gated channel complex",
  "gene": "UniProtKB:P32297",
  "term_id": "GO:0005892",
  "gene_name": "Neuronal acetylcholine receptor subunit alpha-3"
}